enoyl-[acyl-carrier-protein] reductase (NADPH) activity [GO:0141148] (MF) Sources: RHEA:22564 Definition: Catalysis of the reaction: a 2,3-saturated acyl-[ACP] + NADP+ = a (2E)-enoyl-[ACP] + H+ + NADPH. Note: This reaction completes each cycle of fatty acid elongation by catalyzing the stereospecific reduction of the double bond at position 2 of a growing fatty acid chain, while linked to the acyl- carrier protein, in an NADPH-dependent manner. Note that EC has reactions describing the stereo-specificity of the reaction with respect to NADP+ (cf. EC 1.3.1.39, EC 1.3.1.10 and EC 1.3.1.104). Relationships: is a type of enoyl-[acyl-carrier-protein] reductase [NAD(P)H] activity [GO:0016631]